{
  "gene_name": "Pyruvate dehydrogenase E1 component subunit alpha, somatic form, mitochondrial",
  "term_id": "GO:0045254",
  "gene": "UniProtKB:P08559",
  "gene_symbol": "PDHA1",
  "term_label": "pyruvate dehydrogenase complex"
}